cell surface receptor protein tyrosine kinase signaling pathway [GO:0007169] (biological process) Definition: The series of molecular signals initiated by an extracellular ligand binding to a receptor on the surface of the target cell where the receptor possesses tyrosine kinase activity, and ending with the regulation of a downstream cellular process, e.g. transcription. Relationships: is a type of GO:0007167 Sources: GOC:ceb, GOC:signaling Also known as: transmembrane receptor protein serine/threonine kinase signaling pathway, transmembrane receptor protein tyrosine kinase signalling pathway Subtypes: insulin receptor signaling pathway [GO:0008286], torso signaling pathway [GO:0008293], fibroblast growth factor receptor signaling pathway [GO:0008543], brain-derived neurotrophic factor receptor signaling pathway [GO:0031547], glial cell-derived neurotrophic factor receptor signaling pathway [GO:0035860], collagen-activated tyrosine kinase receptor signaling pathway [GO:0038063], vascular endothelial growth factor signaling pathway [GO:0038084], Kit signaling pathway [GO:0038109], ERBB signaling pathway [GO:0038127], sevenless signaling pathway [GO:0045500], platelet-derived growth factor receptor signaling pathway [GO:0048008], insulin-like growth factor receptor signaling pathway [GO:0048009], vascular endothelial growth factor receptor signaling pathway [GO:0048010], neurotrophin TRK receptor signaling pathway [GO:0048011], GO:0048012, ephrin receptor signaling pathway [GO:0048013], GO:0048014, growth hormone receptor signaling pathway [GO:0060396]